{
  "gene": "UniProtKB:Q9BTP6",
  "term_id": "GO:0001227",
  "term_label": "DNA-binding transcription repressor activity, RNA polymerase II-specific",
  "gene_symbol": "ZBED2",
  "gene_name": "Zinc finger BED domain-containing protein 2"
}